{
  "term_id": "UNKNOWN:0002",
  "term_label": "Unknown biological process",
  "gene_name": "Protein phosphatase 1M",
  "gene": "UniProtKB:Q96MI6",
  "gene_symbol": "PPM1M"
}